notochord development [GO:0030903] (biological process) Sources: GOC:dgh Relationships: is a type of embryonic organ development [GO:0048568] Definition: The process whose specific outcome is the progression of the notochord over time, from its formation to the mature structure. The notochord is a mesoderm-derived structure located ventral of the developing nerve cord. In vertebrates, the notochord serves as a core around which other mesodermal cells form the vertebrae. In the most primitive chordates, which lack vertebrae, the notochord persists as a substitute for a vertebral column.